{
  "gene_name": "Lanosterol 14-alpha demethylase",
  "gene_symbol": "CYP51A1",
  "term_id": "UNKNOWN:0003",
  "gene": "UniProtKB:Q16850",
  "term_label": "Unknown cellular component"
}